phosphomethylpyrimidine kinase activity [GO:0008972] (molecular function) Relationships: is_a GO:0016301; is a type of phosphotransferase activity, phosphate group as acceptor [GO:0016776] Definition: Catalysis of the reaction: ATP + 4-amino-2-methyl-5-phosphomethylpyrimidine = ADP + 4-amino-2-methyl-5-diphosphomethylpyrimidine. Sources: EC:2.7.4.7 Also known as: ATP:4-amino-2-methyl-5-phosphomethylpyrimidine phosphotransferase activity, hydroxymethylpyrimidine phosphokinase activity